{
  "gene": "UniProtKB:Q92618",
  "gene_symbol": "ZNF516",
  "term_label": "regulation of DNA-templated transcription",
  "gene_name": "Zinc finger protein 516",
  "term_id": "GO:0006355"
}